3-methyleneoxindole reductase activity [GO:0047567] (molecular function) Also known as: 3-methyl-1,3-dihydroindol-2-one:NADP+ oxidoreductase activity, 3-methyloxindole:NADP+ oxidoreductase activity Sources: EC:1.3.1.17, RHEA:20257 Definition: Catalysis of the reaction: 3-methyloxindole + NADP+ = 3-methyleneoxindole + H+ + NADPH. Relationships: is a type of oxidoreductase activity, acting on the CH-CH group of donors, NAD or NADP as acceptor [GO:0016628]